{
  "gene_name": "Polypeptide N-acetylgalactosaminyltransferase 17",
  "gene": "UniProtKB:Q6IS24",
  "gene_symbol": "GALNT17",
  "term_id": "GO:0004653",
  "term_label": "polypeptide N-acetylgalactosaminyltransferase activity"
}